{
  "gene_name": "Nephrocystin-4",
  "term_label": "protein localization to ciliary transition zone",
  "term_id": "GO:1904491",
  "gene": "UniProtKB:O75161",
  "gene_symbol": "NPHP4"
}